{
  "gene_name": "Phosphatidylinositol 4,5-bisphosphate 3-kinase catalytic subunit beta isoform",
  "gene_symbol": "PIK3CB",
  "term_label": "phosphatidylinositol-3-phosphate biosynthetic process",
  "gene": "UniProtKB:P42338",
  "term_id": "GO:0036092"
}